{
  "term_label": "astrocyte development",
  "gene": "UniProtKB:P06702",
  "term_id": "GO:0014002",
  "gene_name": "Protein S100-A9",
  "gene_symbol": "S100A9"
}